{
  "term_label": "regulation of Rho protein signal transduction",
  "gene": "UniProtKB:Q96HP0",
  "gene_name": "Dedicator of cytokinesis protein 6",
  "term_id": "GO:0035023",
  "gene_symbol": "DOCK6"
}